{
  "term_label": "Unknown molecular function",
  "gene_symbol": "CT47C1",
  "gene_name": "Cancer_testis antigen family 47 member C1",
  "term_id": "UNKNOWN:0001",
  "gene": "UniProtKB:A0A0U1RQG5"
}